{
  "term_label": "cytoplasm",
  "gene_symbol": "TRIM68",
  "gene_name": "E3 ubiquitin-protein ligase TRIM68",
  "gene": "UniProtKB:Q6AZZ1",
  "term_id": "GO:0005737"
}